{
  "term_label": "3-hydroxyisobutyryl-CoA hydrolase activity",
  "gene_name": "3-hydroxyisobutyryl-CoA hydrolase, mitochondrial",
  "term_id": "GO:0003860",
  "gene_symbol": "HIBCH",
  "gene": "UniProtKB:Q6NVY1"
}